mitotic DNA replication leading strand elongation [GO:1903460] (biological process) Also known as: leading strand elongation involved in DNA replication involved in S phase involved in mitotic cell cycle, leading strand elongation involved in DNA replication involved in S-phase involved in mitotic cell cycle, leading strand elongation involved in mitotic DNA replication, leading strand elongation involved in mitotic nuclear cell cycle DNA replication, leading strand elongation involved in DNA replication during S phase involved in mitotic cell cycle, leading strand elongation involved in nuclear cell cycle DNA replication involved in mitotic cell cycle Relationships: is a type of leading strand elongation [GO:0006272]; is a type of DNA strand elongation involved in mitotic DNA replication [GO:1902983] Definition: Any leading strand elongation that is involved in mitotic cell cycle DNA replication. References: PMID:1234 Sources: GOC:TermGenie, GOC:mtg_cell_cycle, GO_REF:0000060